{
  "gene_symbol": "LYPD8",
  "gene": "UniProtKB:Q6UX82",
  "term_label": "defense response to Gram-negative bacterium",
  "term_id": "GO:0050829",
  "gene_name": "Ly6_PLAUR domain-containing protein 8"
}